{
  "gene_name": "Mediator of DNA damage checkpoint protein 1",
  "gene": "UniProtKB:Q14676",
  "gene_symbol": "MDC1",
  "term_label": "histone reader activity",
  "term_id": "GO:0140566"
}